{
  "gene_name": "Lysine-specific demethylase 5A",
  "gene_symbol": "KDM5A",
  "term_id": "GO:0000785",
  "gene": "UniProtKB:P29375",
  "term_label": "chromatin"
}